{
  "gene_name": "MORC family CW-type zinc finger protein 1",
  "gene": "UniProtKB:Q86VD1",
  "term_label": "Unknown biological process",
  "term_id": "UNKNOWN:0002",
  "gene_symbol": "MORC1"
}